{
  "gene_symbol": "RAC1",
  "gene_name": "Ras-related C3 botulinum toxin substrate 1",
  "term_id": "GO:0005886",
  "term_label": "plasma membrane",
  "gene": "UniProtKB:P63000"
}